HslUV protease complex [GO:0009376] (cellular component) Relationships: is a type of cytosolic proteasome complex [GO:0031597] Definition: A protein complex that possesses ATP-dependent protease activity; consists of an ATPase large subunit with homology to other ClpX family ATPases and a peptidase small subunit related to the proteasomal beta-subunits of eukaryotes. In the E. coli complex, a double ring-shaped homohexamer of HslV is capped on each side by a ring-shaped HslU homohexamer. References: PMID:12670962 Sources: GOC:bhm, UniProt:P0A6H5 Also known as: ClpYQ protease complex